{
  "gene": "UniProtKB:P17081",
  "gene_name": "Rho-related GTP-binding protein RhoQ",
  "term_id": "GO:0005525",
  "gene_symbol": "RHOQ",
  "term_label": "GTP binding"
}